{
  "gene": "UniProtKB:P29275",
  "term_label": "plasma membrane",
  "gene_symbol": "ADORA2B",
  "term_id": "GO:0005886",
  "gene_name": "Adenosine receptor A2b"
}